{
  "gene": "UniProtKB:P13164",
  "gene_symbol": "IFITM1",
  "gene_name": "Interferon-induced transmembrane protein 1",
  "term_id": "GO:0034341",
  "term_label": "response to type II interferon"
}